{
  "gene_symbol": "ITGB1BP2",
  "gene_name": "Integrin beta-1-binding protein 2",
  "term_id": "GO:0030018",
  "gene": "UniProtKB:Q9UKP3",
  "term_label": "Z disc"
}